{
  "gene_symbol": "COL27A1",
  "gene": "UniProtKB:Q8IZC6",
  "term_label": "skeletal system development",
  "gene_name": "Collagen alpha-1(XXVII) chain",
  "term_id": "GO:0001501"
}